{
  "term_label": "structural constituent of ribosome",
  "gene_name": "Large ribosomal subunit protein P1",
  "gene": "UniProtKB:P05386",
  "term_id": "GO:0003735",
  "gene_symbol": "RPLP1"
}